{
  "gene_symbol": "TMCC3",
  "gene_name": "Transmembrane and coiled-coil domain protein 3",
  "term_id": "GO:0012505",
  "term_label": "endomembrane system",
  "gene": "UniProtKB:Q9ULS5"
}